{
  "gene_symbol": "PSMD12",
  "gene_name": "26S proteasome non-ATPase regulatory subunit 12",
  "term_label": "Unknown molecular function",
  "term_id": "UNKNOWN:0001",
  "gene": "UniProtKB:O00232"
}